{
  "term_label": "mRNA 3'-UTR binding",
  "gene": "UniProtKB:Q96I24",
  "gene_name": "Far upstream element-binding protein 3",
  "term_id": "GO:0003730",
  "gene_symbol": "FUBP3"
}